{
  "gene_symbol": "CD14",
  "gene_name": "Monocyte differentiation antigen CD14",
  "gene": "UniProtKB:P08571",
  "term_label": "external side of plasma membrane",
  "term_id": "GO:0009897"
}